{
  "term_id": "GO:0005769",
  "gene_symbol": "WASH6P",
  "gene": "UniProtKB:Q9NQA3",
  "term_label": "early endosome",
  "gene_name": "WAS protein family homolog 6"
}